{
  "gene_symbol": "LILRB5",
  "term_id": "GO:0019221",
  "gene": "UniProtKB:O75023",
  "term_label": "cytokine-mediated signaling pathway",
  "gene_name": "Leukocyte immunoglobulin-like receptor subfamily B member 5"
}